6-hydroxynicotinate dehydrogenase activity [GO:0043732] (molecular function) Sources: EC:1.17.3.3, RHEA:22808 Definition: Catalysis of the reaction: 6-hydroxynicotinate + H2O + O2 = 2,6-dihydroxynicotinate + H2O2. Relationships: is a type of oxidoreductase activity, acting on CH or CH2 groups, oxygen as acceptor [GO:0016727] Also known as: 6-hydroxynicotinate hydroxylase activity, 6-hydroxynicotinate:O2 oxidoreductase activity, 6-hydroxynicotinic acid dehydrogenase activity, 6-hydroxynicotinic acid hydroxylase activity